{
  "term_id": "GO:0007254",
  "gene": "UniProtKB:O43318",
  "term_label": "JNK cascade",
  "gene_symbol": "MAP3K7",
  "gene_name": "Mitogen-activated protein kinase kinase kinase 7"
}